{
  "term_label": "D-glucose import",
  "gene": "UniProtKB:Q9BYW1",
  "gene_name": "Solute carrier family 2, facilitated glucose transporter member 11",
  "gene_symbol": "SLC2A11",
  "term_id": "GO:0046323"
}